{
  "gene_symbol": "AURKAIP1",
  "gene": "UniProtKB:Q9NWT8",
  "term_id": "UNKNOWN:0001",
  "term_label": "Unknown molecular function",
  "gene_name": "Small ribosomal subunit protein mS38"
}